{
  "term_id": "GO:0005886",
  "gene_name": "Olfactory receptor 51B2",
  "gene": "UniProtKB:Q9Y5P1",
  "term_label": "plasma membrane",
  "gene_symbol": "OR51B2"
}